notochord regression [GO:0060032] (biological process) Definition: The developmental process in which the structure of the notochord is destroyed in an embryo. Sources: GOC:dph Relationships: is a type of anatomical structure regression [GO:0060033]; BFO_0000050 notochord morphogenesis [GO:0048570]